{
  "term_label": "dense core granule",
  "gene_name": "Synaptotagmin-5",
  "gene_symbol": "SYT5",
  "term_id": "GO:0031045",
  "gene": "UniProtKB:O00445"
}